[isocitrate dehydrogenase (NADP+)] phosphatase activity [GO:0101014] (molecular function) References: PMID:6292732 Sources: MetaCyc:DEPHOSICITDEHASE-RXN Also known as: isocitrate dehydrogenase kinase/phosphatase activity Relationships: is a type of GO:0004721 Definition: Catalysis of the reaction: [isocitrate dehydrogenase] phosphate + H2O = [isocitrate dehydrogenase] + phosphate.